{
  "gene_symbol": "PRORP",
  "term_label": "mitochondrial tRNA 5'-end processing",
  "gene": "UniProtKB:O15091",
  "term_id": "GO:0097745",
  "gene_name": "Mitochondrial ribonuclease P catalytic subunit"
}